retina layer formation [GO:0010842] (biological process) References: PMID:1270266 Sources: GOC:ascb_2009, GOC:dph, GOC:tb Also known as: retinal lamination, retinal layer formation Definition: The process in which the vertebrate retina is organized into three laminae: the outer nuclear layer (ONL), which contains photoreceptor nuclei; the inner nuclear layer (INL), which contains amacrine, bipolar and horizontal cells; and the retinal ganglion cell (RGC) layer. Between the inner and outer nuclear layers, the outer plexiform layer (OPL) contains connections between the photoreceptors and bipolar and horizontal cells. The inner plexiform layer (IPL) is positioned between the INL and the ganglion cell layer and contains the dendrites of RGCs and processes of bipolar and amacrine cells. Spanning all layers of the retina are the radially oriented Mueller glia. Relationships: is a type of GO:0048646; is part of neural retina development [GO:0003407]; is part of retina morphogenesis in camera-type eye [GO:0060042]